{
  "term_label": "plasma membrane",
  "gene": "UniProtKB:Q9ULX7",
  "gene_name": "Carbonic anhydrase 14",
  "gene_symbol": "CA14",
  "term_id": "GO:0005886"
}